response to host iron concentration [GO:0075139] (biological process) Sources: GOC:pamgo_curators Also known as: response of symbiont to host iron concentration Definition: Any process that results in a change in state or activity of the symbiont or its cell (in terms of movement, secretion, enzyme production, gene expression, etc.) as a result of detecting iron concentration in its host organism. The host is defined as the larger of the organisms involved in a symbiotic interaction. Note: Note that this term is used to annotate gene products of the symbiont. Relationships: is a type of response to host [GO:0075136]